interleukin-35 receptor binding [GO:0070748] (molecular function) Definition: Binding to an interleukin-35 receptor. Sources: GOC:add Also known as: IL-35, interleukin-35 receptor ligand Relationships: is a type of cytokine receptor binding [GO:0005126]